{
  "term_id": "GO:0043296",
  "gene": "UniProtKB:Q9ULL8",
  "gene_name": "Protein Shroom4",
  "term_label": "apical junction complex",
  "gene_symbol": "SHROOM4"
}